{
  "term_label": "GTPase activity",
  "term_id": "GO:0003924",
  "gene_symbol": "RAB40A",
  "gene_name": "Ras-related protein Rab-40A",
  "gene": "UniProtKB:Q8WXH6"
}